lysophosphatidic acid receptor activity [GO:0070915] (molecular function) References: PMID:15755723 Sources: GOC:bf, GOC:mah Definition: Combining with the phospholipid derivative lysophosphatidic acid, and transmitting the signal across the membrane by activating an associated G-protein. Relationships: is a type of bioactive lipid receptor activity [GO:0045125]; has part lysophosphatidic acid binding [GO:0035727] Also known as: LPA receptor activity